{
  "gene_symbol": "PLXNA2",
  "term_label": "semaphorin receptor activity",
  "gene": "UniProtKB:O75051",
  "term_id": "GO:0017154",
  "gene_name": "Plexin-A2"
}